dystroglycan binding [GO:0002162] (molecular function) Also known as: alpha-dystroglycan binding, beta-dystroglycan binding Definition: Binding to dystroglycan, a glycoprotein found in non-muscle tissues as well as in muscle tissues, often in association with dystrophin. The native dystroglycan cleaved into two non-covalently associated subunits, alpha (N-terminal) and beta (C-terminal). Relationships: is a type of GO:0005515 Sources: GOC:hjd